{
  "term_label": "Unknown molecular function",
  "gene_name": "Large ribosomal subunit protein mL52",
  "gene_symbol": "MRPL52",
  "gene": "UniProtKB:Q86TS9",
  "term_id": "UNKNOWN:0001"
}